glutathione-cystine transhydrogenase activity [GO:0047141] (molecular function) Also known as: GSH-cystine transhydrogenase, NADPH-dependent GSH-cystine transhydrogenase, glutathione:cystine oxidoreductase Relationships: is a type of oxidoreductase activity, acting on a sulfur group of donors, disulfide as acceptor [GO:0016671] Definition: Catalysis of the reaction: cystine + 2 reduced glutathione = oxidized glutathione + 2 L-cysteine. Sources: EC:1.8.4.4, MetaCyc:1.8.4.4-RXN